{
  "gene": "UniProtKB:P55081",
  "gene_name": "Microfibrillar-associated protein 1",
  "term_id": "GO:0005684",
  "gene_symbol": "MFAP1",
  "term_label": "U2-type spliceosomal complex"
}